protein serine/threonine kinase binding [GO:0120283] (molecular function) References: PMID:28608965 Sources: GOC:krc, GOC:sl Relationships: is a type of protein kinase binding [GO:0019901] Definition: Binding to a protein serine/threonine kinase.